xanthine transmembrane transporter activity [GO:0042907] (molecular function) Sources: GOC:jl Relationships: is_a purine nucleobase transmembrane transporter activity [GO:0005345]; is part of GO:0042906 Definition: Enables the transfer of xanthine from one side of a membrane to the other. Xanthine (2,6-dihydroxypurine) is a purine formed in the metabolic breakdown of guanine, but is not present in nucleic acids.